vestibular calyx terminal [GO:0099096] (cellular component) Relationships: is a type of axon terminus [GO:0043679] Definition: The giant, cup-shaped axon terminal of a vestibular afferent neuron, serving as a post-synaptic contact to a type I hair cell. References: PMID:10706428, PMID:25355208